{
  "gene_name": "T cell receptor beta variable 15 (Fragment)",
  "gene_symbol": "TRBV15",
  "gene": "UniProtKB:A0A087WZ39",
  "term_id": "GO:0007166",
  "term_label": "cell surface receptor signaling pathway"
}